{
  "gene_name": "Chromodomain-helicase-DNA-binding protein 6",
  "gene": "UniProtKB:Q8TD26",
  "gene_symbol": "CHD6",
  "term_label": "DNA binding",
  "term_id": "GO:0003677"
}